{
  "gene": "UniProtKB:Q12959",
  "term_id": "GO:0098839",
  "term_label": "postsynaptic density membrane",
  "gene_symbol": "DLG1",
  "gene_name": "Disks large homolog 1"
}